regulation of toll-like receptor signaling pathway [GO:0034121] (biological process) References: PMID:16551253, PMID:17328678 Sources: GOC:add Relationships: is a type of GO:0062207; regulates toll-like receptor signaling pathway [GO:0002224] Subtypes: negative regulation of toll-like receptor signaling pathway [GO:0034122], positive regulation of toll-like receptor signaling pathway [GO:0034123], regulation of MyD88-dependent toll-like receptor signaling pathway [GO:0034124], regulation of MyD88-independent toll-like receptor signaling pathway [GO:0034127], GO:2000443 Definition: Any process that modulates the frequency, rate, or extent of toll-like receptor signaling pathway. Also known as: regulation of TLR signaling pathway, regulation of toll-like receptor signalling pathway